symmetric neuroblast division [GO:0055058] (biological process) Relationships: is_a neuroblast division [GO:0055057] Definition: The process resulting in the physical partitioning and separation of a neuroblast into two equi-potent daughter cells. Sources: GOC:dph